{
  "term_label": "regulation of transcription by RNA polymerase II",
  "gene_name": "Zinc finger protein 883",
  "gene_symbol": "ZNF883",
  "gene": "UniProtKB:P0CG24",
  "term_id": "GO:0006357"
}